{
  "gene": "UniProtKB:Q9H0K1",
  "gene_name": "Serine_threonine-protein kinase SIK2",
  "term_id": "GO:0004674",
  "gene_symbol": "SIK2",
  "term_label": "protein serine/threonine kinase activity"
}